negative regulation of cardiac muscle hypertrophy [GO:0010614] (BP) Sources: GOC:BHF, GOC:dph, GOC:tb Relationships: is_a GO:0010611; is_a negative regulation of muscle hypertrophy [GO:0014741]; negatively regulates cardiac muscle hypertrophy [GO:0003300] Subtypes: negative regulation of cell growth involved in cardiac muscle cell development [GO:0061052], negative regulation of cardiac muscle hypertrophy in response to stress [GO:1903243] Definition: Any process that decreases the rate, frequency or extent of the enlargement or overgrowth of all or part of the heart due to an increase in size (not length) of individual cardiac muscle fibers, without cell division.